{
  "gene_name": "Peroxiredoxin-4",
  "term_id": "GO:0008379",
  "gene_symbol": "PRDX4",
  "term_label": "thioredoxin peroxidase activity",
  "gene": "UniProtKB:Q13162"
}